xylogalacturonan beta-1,3-xylosyltransferase activity [GO:0102983] (molecular function) Definition: Catalysis of the reaction: UDP-alpha-D-xylose + a homogalacturonan = UDP + 4 H+ + a xylogalacturonan. Relationships: is a type of GO:0016763 Sources: EC:2.4.2.41, GOC:pz